{
  "term_id": "GO:0005886",
  "gene_symbol": "KCNK12",
  "term_label": "plasma membrane",
  "gene": "UniProtKB:Q9HB15",
  "gene_name": "Potassium channel subfamily K member 12"
}